{
  "gene": "UniProtKB:Q9UNQ2",
  "gene_name": "Probable dimethyladenosine transferase",
  "term_label": "rRNA (adenine-N6,N6-)-dimethyltransferase activity",
  "term_id": "GO:0000179",
  "gene_symbol": "DIMT1"
}